{
  "gene": "UniProtKB:Q6R327",
  "term_label": "protein serine/threonine kinase activator activity",
  "term_id": "GO:0043539",
  "gene_symbol": "RICTOR",
  "gene_name": "Rapamycin-insensitive companion of mTOR"
}